regulation of metanephric glomerular mesangial cell proliferation [GO:0072301] (biological process) Definition: Any process that modulates the frequency, rate or extent of metanephric glomerular mesangial cell proliferation. Relationships: is a type of regulation of glomerular mesangial cell proliferation [GO:0072124]; regulates metanephric glomerular mesangial cell proliferation involved in metanephros development [GO:0072262] Subtypes: negative regulation of metanephric glomerular mesangial cell proliferation [GO:0072302], positive regulation of glomerular metanephric mesangial cell proliferation [GO:0072303] Sources: GOC:mtg_kidney_jan10